{
  "gene": "UniProtKB:Q96HM7",
  "gene_symbol": "PCED1B",
  "term_id": "UNKNOWN:0002",
  "term_label": "Unknown biological process",
  "gene_name": "PC-esterase domain-containing protein 1B"
}